regulation of protein sumoylation [GO:0033233] (BP) Also known as: regulation of sumoylation Relationships: is a type of regulation of protein modification by small protein conjugation or removal [GO:1903320]; regulates protein sumoylation [GO:0016925] Subtypes: negative regulation of protein sumoylation [GO:0033234], positive regulation of protein sumoylation [GO:0033235] Sources: GOC:mah Definition: Any process that modulates the frequency, rate or extent of the addition of SUMO groups to a protein.